{
  "gene_name": "Thiamine transporter 2",
  "term_label": "thiamine transmembrane transporter activity",
  "term_id": "GO:0015234",
  "gene_symbol": "SLC19A3",
  "gene": "UniProtKB:Q9BZV2"
}